{
  "term_label": "nucleus",
  "term_id": "GO:0005634",
  "gene_name": "Ubiquitin carboxyl-terminal hydrolase 40",
  "gene": "UniProtKB:Q9NVE5",
  "gene_symbol": "USP40"
}